regulation of phagocytosis, engulfment [GO:0060099] (biological process) Definition: Any process that modulates the frequency, rate or extent of the internalization of bacteria, immune complexes and other particulate matter or of an apoptotic cell by phagocytosis. Subtypes: positive regulation of phagocytosis, engulfment [GO:0060100], negative regulation of phagocytosis, engulfment [GO:0060101], GO:1901074 Sources: GOC:dph Relationships: is a type of regulation of phagocytosis [GO:0050764]; is a type of regulation of membrane invagination [GO:1905153]; regulates phagocytosis, engulfment [GO:0006911]